{
  "term_id": "GO:0005576",
  "gene": "UniProtKB:Q9NQ38",
  "gene_name": "Serine protease inhibitor Kazal-type 5",
  "term_label": "extracellular region",
  "gene_symbol": "SPINK5"
}